{
  "term_id": "GO:0032050",
  "gene_symbol": "GPR107",
  "gene_name": "Protein GPR107",
  "term_label": "clathrin heavy chain binding",
  "gene": "UniProtKB:Q5VW38"
}